photosystem I antenna complex [GO:0009782] (cellular component) Relationships: is a type of GO:0098796; is part of photosystem I [GO:0009522] Sources: GOC:jid, ISBN:0716731363 Definition: The antenna complex of photosystem I. A photosystem has two closely linked components, an antenna containing light-absorbing pigments and a reaction center. Each antenna contains one or more light-harvesting complexes (LHCs).